tectum [GO:0043676] (cellular component) Definition: The layer of sexine which forms a roof over the columella, granules or other infratectal elements. References: PMID:33706055 Relationships: is a type of GO:0110165; is part of sexine [GO:0043673] Also known as: sexine 2